{
  "gene_symbol": "TOPAZ1",
  "term_id": "GO:0048137",
  "gene_name": "Protein TOPAZ1",
  "gene": "UniProtKB:Q8N9V7",
  "term_label": "spermatocyte division"
}